{
  "term_label": "Unknown biological process",
  "gene": "UniProtKB:Q9NS37",
  "gene_name": "CREB_ATF bZIP transcription factor",
  "term_id": "UNKNOWN:0002",
  "gene_symbol": "CREBZF"
}